{
  "gene_symbol": "HIPK4",
  "term_id": "GO:0004674",
  "gene_name": "Homeodomain-interacting protein kinase 4",
  "term_label": "protein serine/threonine kinase activity",
  "gene": "UniProtKB:Q8NE63"
}